nuclear DNA-directed RNA polymerase complex [GO:0055029] (cellular component) Definition: A protein complex, located in the nucleus, that possesses DNA-directed RNA polymerase activity. Sources: GOC:mtg_sensu Relationships: is a type of DNA-directed RNA polymerase complex [GO:0000428]; is a type of GO:0140513; is part of nucleoplasm [GO:0005654] Subtypes: alpha DNA polymerase:primase complex [GO:0005658], RNA polymerase II, core complex [GO:0005665], RNA polymerase II, holoenzyme [GO:0016591]